{
  "gene": "UniProtKB:Q8NER5",
  "gene_symbol": "ACVR1C",
  "term_label": "cellular response to growth factor stimulus",
  "gene_name": "Activin receptor type-1C",
  "term_id": "GO:0071363"
}